{
  "term_label": "peroxisome",
  "gene_name": "KICSTOR complex protein SZT2",
  "term_id": "GO:0005777",
  "gene": "UniProtKB:Q5T011",
  "gene_symbol": "SZT2"
}